{
  "term_label": "protein serine/threonine kinase activity",
  "gene_name": "Mitogen-activated protein kinase 6",
  "gene_symbol": "MAPK6",
  "term_id": "GO:0004674",
  "gene": "UniProtKB:Q16659"
}